{
  "gene_name": "DC-STAMP domain-containing protein 2",
  "term_id": "UNKNOWN:0003",
  "gene_symbol": "DCST2",
  "gene": "UniProtKB:Q5T1A1",
  "term_label": "Unknown cellular component"
}